{
  "gene": "UniProtKB:Q9H2X9",
  "term_id": "GO:0005886",
  "term_label": "plasma membrane",
  "gene_name": "Solute carrier family 12 member 5",
  "gene_symbol": "SLC12A5"
}